{
  "gene": "UniProtKB:Q13705",
  "gene_symbol": "ACVR2B",
  "gene_name": "Activin receptor type-2B",
  "term_id": "GO:0032924",
  "term_label": "activin receptor signaling pathway"
}